{
  "term_label": "glucose metabolic process",
  "term_id": "GO:0006006",
  "gene_name": "Fibrillin-3",
  "gene_symbol": "FBN3",
  "gene": "UniProtKB:Q75N90"
}